calcium activated phosphatidylcholine scrambling [GO:0061590] (biological process) Definition: The movement of a population of phosphatidylcholine molecules from one leaflet of the plasma membrane bilayer to the opposite leaflet as a result of a calcium stimulus. Relationships: is a type of calcium activated phospholipid scrambling [GO:0061588] References: PMID:23532839 Sources: GOC:krc